{
  "gene_name": "LHFPL tetraspan subfamily member 7 protein",
  "gene": "UniProtKB:Q6ICI0",
  "term_label": "Unknown molecular function",
  "gene_symbol": "LHFPL7",
  "term_id": "UNKNOWN:0001"
}